{
  "gene_name": "Endophilin-A3",
  "term_id": "GO:0061024",
  "gene": "UniProtKB:Q99963",
  "gene_symbol": "SH3GL3",
  "term_label": "membrane organization"
}